endocardial cell differentiation [GO:0060956] (biological process) Sources: GOC:mtg_heart Definition: The process in which a relatively unspecialized cell acquires the specialized structural and/or functional features of an endocardial cell. An endocardial cell is a specialized endothelial cell that makes up the endocardium portion of the heart. The endocardium is the innermost layer of tissue of the heart, and lines the heart chambers. Relationships: is a type of GO:0003348; is part of endocardium development [GO:0003157]